{
  "gene_name": "Binder of sperm protein homolog 1",
  "gene_symbol": "BSPH1",
  "term_id": "GO:0048240",
  "term_label": "sperm capacitation",
  "gene": "UniProtKB:Q075Z2"
}